{
  "gene": "UniProtKB:P08237",
  "term_label": "fructose-6-phosphate binding",
  "term_id": "GO:0070095",
  "gene_symbol": "PFKM",
  "gene_name": "ATP-dependent 6-phosphofructokinase, muscle type"
}